{
  "term_label": "CXCR4 chemokine receptor binding",
  "gene_symbol": "TFF2",
  "gene_name": "Trefoil factor 2",
  "gene": "UniProtKB:Q03403",
  "term_id": "GO:0031723"
}